{
  "term_id": "UNKNOWN:0002",
  "gene_name": "TBC1 domain family member 16",
  "term_label": "Unknown biological process",
  "gene": "UniProtKB:Q8TBP0",
  "gene_symbol": "TBC1D16"
}